vesicle scission involved in clathrin-mediated endocytosis [GO:0099052] (biological process) References: PMID:21779028 Definition: The membrane scission process that is the final step in the formation of a clathrin-coated endocytic vesicle: separation from the plasma membrane. Relationships: is a type of GO:0099051; is part of clathrin-dependent endocytosis [GO:0072583] Note: Like other vesicle scission events this involves dynamin. At least some of the dynamin recruiting factors are distinct to scission of clathrin-coated vesicles (PMID:21779028).